{
  "term_label": "Unknown molecular function",
  "gene_symbol": "LINC00523",
  "gene_name": "Putative uncharacterized protein encoded by LINC00523",
  "gene": "UniProtKB:Q86TU6",
  "term_id": "UNKNOWN:0001"
}